electrosensory lateral line system development [GO:0048926] (biological process) Definition: The process whose specific outcome is the progression of the electrosensory lateral line system over time, from its formation to the mature structure. Sources: GOC:dgh Relationships: is a type of lateral line system development [GO:0048925]